{
  "gene_name": "Protein S100-A12",
  "gene": "UniProtKB:P80511",
  "gene_symbol": "S100A12",
  "term_id": "GO:0050786",
  "term_label": "RAGE receptor binding"
}